{
  "gene": "UniProtKB:Q9H0Y0",
  "term_id": "UNKNOWN:0003",
  "gene_name": "Ubiquitin-like-conjugating enzyme ATG10",
  "term_label": "Unknown cellular component",
  "gene_symbol": "ATG10"
}